{
  "gene": "UniProtKB:Q9GZV3",
  "gene_symbol": "SLC5A7",
  "term_label": "acetylcholine biosynthetic process",
  "term_id": "GO:0008292",
  "gene_name": "High affinity choline transporter 1"
}